{
  "term_label": "cell adhesion molecule binding",
  "gene_name": "Protocadherin alpha-4",
  "gene_symbol": "PCDHA4",
  "term_id": "GO:0050839",
  "gene": "UniProtKB:Q9UN74"
}